glucan endo-1,3-alpha-glucosidase activity [GO:0051118] (molecular function) Relationships: is a type of alpha-glucosidase activity [GO:0090599] Also known as: 1,3(1,3;1,4)-alpha-D-glucan 3-glucanohydrolase activity, cariogenanase activity, cariogenase activity, endo-(1->3)-alpha-glucanase activity, endo-1,3-alpha-D-glucanase activity, endo-1,3-alpha-glucanase activity, mutanase activity Definition: Catalysis of the endohydrolysis of (1->3)-alpha-D-glucosidic linkages in isolichenin, pseudonigeran and nigeran. Sources: EC:3.2.1.59